negative regulation of trypanothione biosynthetic process [GO:1905723] (biological process) Also known as: down regulation of trypanothione anabolism, down regulation of trypanothione biosynthesis, down regulation of trypanothione biosynthetic process, down regulation of trypanothione formation, down regulation of trypanothione synthesis, down-regulation of trypanothione anabolism, down-regulation of trypanothione biosynthesis, down-regulation of trypanothione biosynthetic process, down-regulation of trypanothione formation, down-regulation of trypanothione synthesis, downregulation of trypanothione anabolism, downregulation of trypanothione biosynthesis, downregulation of trypanothione biosynthetic process, downregulation of trypanothione formation, downregulation of trypanothione synthesis, negative regulation of trypanothione anabolism, negative regulation of trypanothione biosynthesis, negative regulation of trypanothione formation, negative regulation of trypanothione synthesis, inhibition of trypanothione anabolism, inhibition of trypanothione biosynthesis, inhibition of trypanothione biosynthetic process, inhibition of trypanothione formation, inhibition of trypanothione synthesis Relationships: is a type of negative regulation of biosynthetic process [GO:0009890]; is a type of GO:1905722; negatively regulates trypanothione biosynthetic process [GO:0019342] Definition: Any process that stops, prevents or reduces the frequency, rate or extent of trypanothione biosynthetic process. References: PMID:18949025 Sources: GOC:TermGenie, GO_REF:0000058